{
  "term_id": "GO:0005737",
  "gene_name": "Cyclin-dependent kinase 18",
  "term_label": "cytoplasm",
  "gene": "UniProtKB:Q07002",
  "gene_symbol": "CDK18"
}